pyrimidine nucleoside diphosphate biosynthetic process [GO:0009139] (biological process) Sources: GOC:go_curators, ISBN:0198506732 Also known as: pyrimidine nucleoside diphosphate anabolism, pyrimidine nucleoside diphosphate biosynthesis, pyrimidine nucleoside diphosphate formation, pyrimidine nucleoside diphosphate synthesis Definition: The chemical reactions and pathways resulting in the formation of pyrimidine nucleoside diphosphate, a compound consisting of a pyrimidine base linked to a ribose or deoxyribose sugar esterified with diphosphate on the sugar. Subtypes: GO:0009194, GO:0009197 Relationships: is a type of GO:0009133; is a type of pyrimidine nucleoside diphosphate metabolic process [GO:0009138]